{
  "gene": "UniProtKB:Q5H9R4",
  "gene_name": "Armadillo repeat-containing X-linked protein 4",
  "gene_symbol": "ARMCX4",
  "term_label": "Unknown cellular component",
  "term_id": "UNKNOWN:0003"
}